{
  "gene_name": "ATP-binding cassette sub-family G member 4",
  "gene": "UniProtKB:Q9H172",
  "gene_symbol": "ABCG4",
  "term_id": "GO:0042632",
  "term_label": "cholesterol homeostasis"
}